{
  "gene_name": "Small G protein signaling modulator 3",
  "gene_symbol": "SGSM3",
  "gene": "UniProtKB:Q96HU1",
  "term_id": "UNKNOWN:0003",
  "term_label": "Unknown cellular component"
}